{
  "term_id": "GO:0071218",
  "gene_name": "DnaJ homolog subfamily B member 14",
  "term_label": "cellular response to misfolded protein",
  "gene": "UniProtKB:Q8TBM8",
  "gene_symbol": "DNAJB14"
}